proteasome-activating activity [GO:0036402] (molecular function) Relationships: is a type of GO:0120544; is a type of ATP-dependent activity [GO:0140657]; is part of proteasomal protein catabolic process [GO:0010498] Also known as: ATPase involved in positive regulation of proteasomal protein catabolic process, proteasomal ATPase activity, proteasome-activating ATPase activity, proteasome channel gating activity, proteasome channel opening activity References: PMID:11430818 Sources: GOC:rb Definition: Catalysis of the reaction: ATP + H2O = ADP + phosphate, which promotes unfolding of protein substrates, and channel opening of the core proteasome.